regulation of cellular response to stress [GO:0080135] (biological process) Relationships: is a type of regulation of cellular process [GO:0050794]; is a type of regulation of response to stress [GO:0080134]; regulates cellular response to stress [GO:0033554] Definition: Any process that modulates the frequency, rate or extent of a cellular response to stress. Cellular response to stress is a change in state or activity of a cell (in terms of movement, secretion, enzyme production, gene expression, etc.) as a result of a stimulus indicating the organism is under stress. The stress is usually, but not necessarily, exogenous (e.g. temperature, humidity, ionizing radiation). Subtypes: GO:0006282, regulation of plant-type hypersensitive response [GO:0010363], GO:0010516, regulation of eIF2 alpha phosphorylation by heme [GO:0010999], GO:0043516, regulation of aggregation involved in sorocarp development [GO:0060176], regulation of eIF2 alpha phosphorylation by dsRNA [GO:0060735], GO:0060905, regulation of stress-activated protein kinase signaling cascade [GO:0070302], GO:0070570, GO:0080136, regulation of cellular response to osmotic stress [GO:0106049], regulation of cellular response to phosphate starvation [GO:0140255], negative regulation of GDF15-GFRAL signaling pathway [GO:0160145], regulation of cellular response to heat [GO:1900034], GO:1900037, regulation of cellular response to oxidative stress [GO:1900407], regulation of cellular response to iron ion starvation [GO:1901966], regulation of intrinsic apoptotic signaling pathway in response to DNA damage [GO:1902229], regulation of cellular response to amino acid starvation [GO:1903832], regulation of error-prone translesion synthesis [GO:1904331], regulation of telomere maintenance in response to DNA damage [GO:1904505], regulation of cellular response to glucose starvation [GO:1904547], regulation of nitrosative stress-induced intrinsic apoptotic signaling pathway [GO:1905258], regulation of response to endoplasmic reticulum stress [GO:1905897], GO:2000001, regulation of SREBP signaling pathway [GO:2000638] Sources: GOC:dhl